{
  "term_label": "Unknown cellular component",
  "gene_name": "Protein FAM25A",
  "term_id": "UNKNOWN:0003",
  "gene_symbol": "FAM25A",
  "gene": "UniProtKB:B3EWG3"
}